{
  "gene_name": "Extracellular sulfatase Sulf-2",
  "gene_symbol": "SULF2",
  "term_label": "negative regulation of fibroblast growth factor receptor signaling pathway",
  "term_id": "GO:0040037",
  "gene": "UniProtKB:Q8IWU5"
}